{
  "term_label": "neuron projection",
  "gene_symbol": "STMN3",
  "gene_name": "Stathmin-3",
  "gene": "UniProtKB:Q9NZ72",
  "term_id": "GO:0043005"
}